streptomycin 3''-kinase activity [GO:0050299] (molecular function) Also known as: ATP:streptomycin 3''-phosphotransferase activity, streptomycin 3''-kinase (phosphorylating), streptomycin 3''-phosphotransferase activity Relationships: is a type of aminoglycoside phosphotransferase activity [GO:0034071] Sources: EC:2.7.1.87, RHEA:18377 Definition: Catalysis of the reaction: ATP + streptomycin = ADP + 2 H+ + streptomycin 3''-phosphate.